positive regulation of T cell homeostatic proliferation [GO:0042103] (biological process) Definition: Any process that activates or increases the rate or extent of resting T cell proliferation. Sources: GOC:jl Also known as: positive regulation of T lymphocyte homeostatic proliferation, positive regulation of T-cell homeostatic proliferation, positive regulation of T-lymphocyte homeostatic proliferation, positive regulation of resting T cell proliferation, up regulation of T cell homeostatic proliferation, up-regulation of T cell homeostatic proliferation, upregulation of T cell homeostatic proliferation, activation of T cell homeostatic proliferation, stimulation of T cell homeostatic proliferation Relationships: is a type of positive regulation of T cell proliferation [GO:0042102]; is a type of GO:0046013; RO_0002213 T cell homeostatic proliferation [GO:0001777]